{
  "term_id": "GO:0060397",
  "gene_symbol": "STAT5B",
  "term_label": "growth hormone receptor signaling pathway via JAK-STAT",
  "gene": "UniProtKB:P51692",
  "gene_name": "Signal transducer and activator of transcription 5B"
}